{
  "gene": "UniProtKB:O60883",
  "gene_name": "G-protein coupled receptor 37-like 1",
  "gene_symbol": "GPR37L1",
  "term_label": "positive regulation of MAPK cascade",
  "term_id": "GO:0043410"
}